{
  "gene": "UniProtKB:Q9HBI6",
  "gene_symbol": "CYP4F11",
  "term_id": "UNKNOWN:0001",
  "gene_name": "Cytochrome P450 4F11",
  "term_label": "Unknown molecular function"
}